{
  "gene_symbol": "FAM166B",
  "term_id": "UNKNOWN:0003",
  "term_label": "Unknown cellular component",
  "gene_name": "Protein FAM166B",
  "gene": "UniProtKB:A8MTA8"
}